{
  "gene_symbol": "PIANP",
  "gene_name": "PILR alpha-associated neural protein",
  "term_id": "GO:0016020",
  "gene": "UniProtKB:Q8IYJ0",
  "term_label": "membrane"
}